{
  "term_label": "Unknown biological process",
  "gene_name": "Filamin-B",
  "gene_symbol": "FLNB",
  "term_id": "UNKNOWN:0002",
  "gene": "UniProtKB:O75369"
}